{
  "term_label": "innate immune response",
  "term_id": "GO:0045087",
  "gene_name": "E3 ubiquitin-protein ligase TRIM48",
  "gene": "UniProtKB:Q8IWZ4",
  "gene_symbol": "TRIM48"
}